{
  "gene": "UniProtKB:O60810",
  "gene_name": "PRAME family member 4",
  "term_id": "GO:1990756",
  "gene_symbol": "PRAMEF4",
  "term_label": "ubiquitin-like ligase-substrate adaptor activity"
}